regulation of chylomicron remnant clearance [GO:0090320] (biological process) Definition: Any process that modulates the rate, frequency or extent of chylomicron remnant clearance. Chylomicron clearance is the process in which a chylomicron remnant is removed from the blood via receptor-mediated endocytosis into liver cells and its constituent parts degraded. Subtypes: positive regulation of chylomicron remnant clearance [GO:0090321] Sources: GOC:tb Relationships: is a type of regulation of lipoprotein particle clearance [GO:0010984]; regulates chylomicron remnant clearance [GO:0034382]